{
  "term_label": "dGTP catabolic process",
  "gene_name": "Nucleotide triphosphate diphosphatase NUDT15",
  "term_id": "GO:0006203",
  "gene_symbol": "NUDT15",
  "gene": "UniProtKB:Q9NV35"
}